{
  "term_label": "microtubule binding",
  "gene_name": "Proline_serine-rich coiled-coil protein 1",
  "gene": "UniProtKB:Q6PGN9",
  "gene_symbol": "PSRC1",
  "term_id": "GO:0008017"
}